rRNA (adenine(2503)-C2-)-methyltransferase activity [GO:0070040] (molecular function) Relationships: is a type of C-methyltransferase activity [GO:0008169]; is a type of rRNA (adenine) methyltransferase activity [GO:0016433] References: PMID:20007606, PMID:20184321, PMID:21368151, PMID:21415317, PMID:21527678 Sources: GOC:imk, RHEA:42916 Definition: Catalysis of the reaction: adenosine2503 in 23S rRNA + 2 reduced [2Fe-2S]-[ferredoxin] + 2 S-adenosyl-L-methionine = 2-methyladenosine2503 in 23S rRNA + 5'-deoxyadenosine + L-methionine + 2 oxidized [2Fe-2S]-[ferredoxin] + S-adenosyl-L-homocysteine. Also known as: rRNA (adenine-C2-)-methyltransferase activity